{
  "gene_name": "G patch domain-containing protein 3",
  "term_id": "GO:0045893",
  "term_label": "positive regulation of DNA-templated transcription",
  "gene": "UniProtKB:Q96I76",
  "gene_symbol": "GPATCH3"
}